{
  "gene": "UniProtKB:Q13641",
  "term_label": "Unknown molecular function",
  "gene_symbol": "TPBG",
  "term_id": "UNKNOWN:0001",
  "gene_name": "Trophoblast glycoprotein"
}